{
  "term_label": "animal organ development",
  "term_id": "GO:0048513",
  "gene": "UniProtKB:P31314",
  "gene_name": "T-cell leukemia homeobox protein 1",
  "gene_symbol": "TLX1"
}